{
  "term_id": "GO:0030527",
  "term_label": "structural constituent of chromatin",
  "gene": "UniProtKB:P0C0S8",
  "gene_name": "Histone H2A type 1",
  "gene_symbol": "H2AC17"
}